{
  "gene": "UniProtKB:Q9P2D1",
  "gene_symbol": "CHD7",
  "term_id": "GO:0042472",
  "gene_name": "Chromodomain-helicase-DNA-binding protein 7",
  "term_label": "inner ear morphogenesis"
}